{
  "term_id": "GO:0005604",
  "gene_name": "Collagen alpha-1(XV) chain",
  "gene": "UniProtKB:P39059",
  "gene_symbol": "COL15A1",
  "term_label": "basement membrane"
}